{
  "gene_symbol": "CPNE8",
  "term_id": "GO:0005544",
  "gene_name": "Copine-8",
  "term_label": "calcium-dependent phospholipid binding",
  "gene": "UniProtKB:Q86YQ8"
}